{
  "term_id": "GO:0031594",
  "gene_name": "Synaptogyrin-3",
  "term_label": "neuromuscular junction",
  "gene": "UniProtKB:O43761",
  "gene_symbol": "SYNGR3"
}